symbiont-mediated modulation of host ethylene-mediated defense response [GO:0052084] (biological process) Also known as: modulation by organism of defense-related ethylene-mediated signal transduction pathway in other organism involved in symbiotic interaction, modulation by organism of ethylene-mediated defense response of other organism involved in symbiotic interaction, modulation by symbiont of defense-related host ethylene-mediated signal transduction pathway, modulation by symbiont of host ethylene-mediated defense response Definition: Any process in which a symbiont modulates the frequency, rate or extent of the ethylene-mediated defense response of the host organism. The host is defined as the larger of the organisms involved in a symbiotic interaction. Subtypes: symbiont-mediated suppression of host ethylene-mediated defense response [GO:0052005] Sources: GOC:mtg_pamgo_17jul06 Relationships: is a type of symbiont-mediated perturbation of host defense response [GO:0052031]